{
  "gene_name": "Sulfate transporter",
  "gene": "UniProtKB:P50443",
  "term_id": "GO:1902358",
  "gene_symbol": "SLC26A2",
  "term_label": "sulfate transmembrane transport"
}